neutrophil extravasation [GO:0072672] (biological process) Definition: The migration of a neutrophil from the blood vessels into the surrounding tissue. Sources: CL:0000775, GOC:BHF Relationships: is_a GO:0045123; is a type of neutrophil migration [GO:1990266] Regulation: regulated by GO:2000389; negatively regulated by negative regulation of neutrophil extravasation [GO:2000390]; positively regulated by positive regulation of neutrophil extravasation [GO:2000391]